{
  "gene": "UniProtKB:A0A075B6I3",
  "gene_symbol": "IGLV11-55",
  "gene_name": "Probable non-functional immunoglobulin lambda variable 11-55",
  "term_label": "Unknown molecular function",
  "term_id": "UNKNOWN:0001"
}